{
  "gene_symbol": "CIB3",
  "gene": "UniProtKB:Q96Q77",
  "gene_name": "Calcium and integrin-binding family member 3",
  "term_label": "Unknown cellular component",
  "term_id": "UNKNOWN:0003"
}